{
  "gene_name": "Killer cell lectin-like receptor subfamily F member 1",
  "term_label": "Unknown biological process",
  "term_id": "UNKNOWN:0002",
  "gene": "UniProtKB:Q9NZS2",
  "gene_symbol": "KLRF1"
}